{
  "gene": "UniProtKB:Q5VSP4",
  "gene_name": "Putative lipocalin 1-like protein 1",
  "term_id": "UNKNOWN:0002",
  "gene_symbol": "LCN1P1",
  "term_label": "Unknown biological process"
}